{
  "term_id": "UNKNOWN:0001",
  "gene_name": "Family with sequence similarity 90 member A3, pseudogene",
  "gene_symbol": "FAM90A3P",
  "term_label": "Unknown molecular function",
  "gene": "UniProtKB:A0A8V8TPE2"
}